Golgi membrane [GO:0000139] (cellular component) Definition: The lipid bilayer surrounding any of the compartments of the Golgi apparatus. Sources: GOC:mah Relationships: is a type of bounding membrane of organelle [GO:0098588]; is part of Golgi apparatus [GO:0005794] Also known as: Golgi apparatus membrane